{
  "term_id": "GO:0006357",
  "term_label": "regulation of transcription by RNA polymerase II",
  "gene_symbol": "ZNF586",
  "gene": "UniProtKB:Q9NXT0",
  "gene_name": "Zinc finger protein 586"
}